{
  "gene_symbol": "SLC35A3",
  "term_label": "UDP-galactose transmembrane transporter activity",
  "term_id": "GO:0005459",
  "gene": "UniProtKB:Q9Y2D2",
  "gene_name": "UDP-N-acetylglucosamine transporter"
}